regulation of blastocyst development [GO:0120222] (BP) References: PMID:29593216 Sources: GOC:krc Definition: Any process that modulates the frequency, rate or extent of blastocyst development. Relationships: is a type of regulation of developmental process [GO:0050793]; regulates blastocyst development [GO:0001824]